lateral line ganglion development [GO:0048890] (biological process) Definition: The process whose specific outcome is the progression of the lateral line ganglion over time, from its formation to the mature structure. The lateral line ganglion develops from cranial ectodermal placodes situated between the eye and ear and behind the ear. Also known as: gLL ganglion development Subtypes: anterior lateral line ganglion development [GO:0048907], GO:0048917 Sources: ISBN:0125296509, ISBN:0387968377 Relationships: is a type of cranial ganglion development [GO:0061550]; is part of GO:0007422; is part of lateral line system development [GO:0048925]